{
  "gene_name": "Protein furry homolog",
  "term_label": "cell cortex",
  "gene": "UniProtKB:Q5TBA9",
  "gene_symbol": "FRY",
  "term_id": "GO:0005938"
}